{
  "gene": "UniProtKB:Q12800",
  "gene_name": "Alpha-globin transcription factor CP2",
  "term_label": "RNA polymerase II cis-regulatory region sequence-specific DNA binding",
  "gene_symbol": "TFCP2",
  "term_id": "GO:0000978"
}